protein localization to basolateral plasma membrane [GO:1903361] (biological process) Also known as: basolateral protein localization, protein localisation in basolateral plasma membrane, protein localisation to basolateral plasma membrane, protein localization in basolateral plasma membrane Definition: Any process in which a protein is transported to, or maintained in, basolateral regions of the plasma membrane. Regulation: RO_0002211 by regulation of protein localization to basolateral plasma membrane [GO:1904508]; negatively regulated by negative regulation of protein localization to basolateral plasma membrane [GO:1904509]; positively regulated by positive regulation of protein localization to basolateral plasma membrane [GO:1904510] References: PMID:24785082, PMID:9425351 Sources: GOC:TermGenie, GOC:kmv, GO_REF:0000087 Relationships: is a type of protein localization to membrane [GO:0072657]; is a type of protein localization to cell periphery [GO:1990778]